trisaccharide binding [GO:0048031] (molecular function) Subtypes: GO:0044583 Relationships: is a type of oligosaccharide binding [GO:0070492] Sources: GOC:jid Definition: Binding to a trisaccharide. Trisaccharides are sugars composed of three monosaccharide units.